{
  "term_id": "UNKNOWN:0002",
  "gene": "UniProtKB:Q7Z404",
  "gene_name": "Transmembrane channel-like protein 4",
  "gene_symbol": "TMC4",
  "term_label": "Unknown biological process"
}